{
  "gene": "UniProtKB:Q8TF27",
  "term_label": "GTPase activity",
  "gene_name": "Arf-GAP with GTPase, ANK repeat and PH domain-containing protein 11",
  "gene_symbol": "AGAP11",
  "term_id": "GO:0003924"
}